{
  "gene_name": "Probable G-protein coupled receptor 19",
  "gene_symbol": "GPR19",
  "gene": "UniProtKB:Q15760",
  "term_label": "G protein-coupled receptor signaling pathway",
  "term_id": "GO:0007186"
}